{
  "gene": "UniProtKB:O43541",
  "term_id": "GO:0030154",
  "gene_symbol": "SMAD6",
  "term_label": "cell differentiation",
  "gene_name": "Mothers against decapentaplegic homolog 6"
}